ATP/ADP dimethylallyltransferase activity [GO:0052622] (molecular function) Definition: Catalysis of the reaction: delta(2)-isopentenyl diphosphate + ATP = diphosphate + N6-(delta(2)-isopentenyl)adenosine 5'-triphosphate. Also known as: adenylate isopentenyltransferase activity, cytokinin synthase activity, ADP/ATP dimethylallyltransferase activity, adenylate dimethylallyltransferase (ADP/ATP-dependent) activity, adenylate dimethylallyltransferase (ATP/ADP-dependent) activity, 2-isopentenyl-diphosphate:ADP 2-isopentenyltransferase activity, 2-isopentenyl-diphosphate:ADP delta2-isopentenyltransferase activity, 2-isopentenyl-diphosphate:ATP 2-isopentenyltransferase activity, 2-isopentenyl-diphosphate:ATP delta2-isopentenyltransferase activity, ADP dimethylallyltransferase activity, ADP isopentenyltransferase activity, ATP dimethylallyltransferase activity, ATP isopentenyltransferase activity, dimethylallyl-diphosphate:ADP dimethylallyltransferase activity, dimethylallyl-diphosphate:ATP dimethylallyltransferase activity Relationships: is a type of transferase activity, transferring alkyl or aryl (other than methyl) groups [GO:0016765] Sources: EC:2.5.1.112